{
  "term_id": "GO:0006656",
  "term_label": "phosphatidylcholine biosynthetic process",
  "gene_symbol": "LPCAT3",
  "gene_name": "Lysophospholipid acyltransferase 5",
  "gene": "UniProtKB:Q6P1A2"
}